{
  "gene_symbol": "PCDH7",
  "gene_name": "Protocadherin-7",
  "gene": "UniProtKB:O60245",
  "term_label": "cell adhesion",
  "term_id": "GO:0007155"
}